succinyl-CoA:oxalate CoA-transferase [GO:0050161] (molecular function) Definition: Catalysis of the reaction: oxalate + succinyl-CoA = oxalyl-CoA + succinate. Also known as: oxalate CoA-transferase activity, oxalate coenzyme A-transferase activity, succinyl-CoA:oxalate CoA-transferase activity, succinyl-beta-ketoacyl-CoA transferase activity Sources: EC:2.8.3.2, RHEA:23588 Relationships: is a type of GO:0008410